negative regulation of aggregation involved in sorocarp development [GO:0110014] (biological process) References: PMID:28257811 Sources: GOC:rjd Definition: Any process that decreases the frequency, rate or extent of aggregation involved in sorocarp development. Aggregation involved in sorocarp development is the process whose specific outcome is the progression of the aggregate over time, from its formation to the point when a slug is formed. Aggregate development begins in response to starvation and continues by the chemoattractant-mediated movement of cells toward each other. The aggregate is a multicellular structure that gives rise to the slug. Relationships: is a type of GO:0032108; is a type of negative regulation of cellular process [GO:0048523]; is a type of GO:0051093; is_a GO:0060176; negatively regulates aggregation involved in sorocarp development [GO:0031152]